{
  "term_label": "Unknown molecular function",
  "gene_name": "Aurora kinase A and ninein-interacting protein",
  "gene_symbol": "AUNIP",
  "term_id": "UNKNOWN:0001",
  "gene": "UniProtKB:Q9H7T9"
}